{
  "term_label": "synapse",
  "gene_name": "Sodium-dependent serotonin transporter",
  "term_id": "GO:0045202",
  "gene_symbol": "SLC6A4",
  "gene": "UniProtKB:P31645"
}